interleukin-10 binding [GO:0019969] (molecular function) Sources: GOC:jl Also known as: IL-10 binding Relationships: is a type of growth factor binding [GO:0019838]; is_a GO:0019955 Definition: Binding to interleukin-10.